{
  "term_id": "GO:0005654",
  "gene_name": "Protein TASOR",
  "gene_symbol": "TASOR",
  "term_label": "nucleoplasm",
  "gene": "UniProtKB:Q9UK61"
}